{
  "term_id": "GO:0006338",
  "gene": "UniProtKB:Q8TDI0",
  "term_label": "chromatin remodeling",
  "gene_name": "Chromodomain-helicase-DNA-binding protein 5",
  "gene_symbol": "CHD5"
}